abscisic acid glucose ester beta-glucosidase activity [GO:0051993] (molecular function) Definition: Catalysis of the reaction: abscisic acid glucose ester + H2O = abscisic acid + beta-D-glucose. References: PMID:16990135 Also known as: ABA-GE beta-glucosidase activity Relationships: is a type of beta-glucosidase activity [GO:0008422]